{
  "gene": "UniProtKB:Q9UFW8",
  "gene_name": "CGG triplet repeat-binding protein 1",
  "term_label": "regulation of gene expression",
  "gene_symbol": "CGGBP1",
  "term_id": "GO:0010468"
}